oxidoreductase activity, acting on diphenols and related substances as donors, with copper protein as acceptor [GO:0052880] (molecular function) Sources: GOC:jl Subtypes: plastoquinol--plastocyanin reductase activity [GO:0009496] Definition: Catalysis of an oxidation-reduction (redox) reaction in which a diphenol, or related compound, acts as a hydrogen or electron donor and reduces a copper protein. Relationships: is a type of GO:0016679